positive regulation of filopodium assembly [GO:0051491] (biological process) Sources: GOC:ai, GOC:dph, GOC:tb Definition: Any process that activates or increases the frequency, rate or extent of the assembly of a filopodium, a thin, stiff protrusion extended by the leading edge of a motile cell such as a crawling fibroblast or amoeba, or an axonal growth cone. Relationships: is a type of regulation of filopodium assembly [GO:0051489]; is a type of positive regulation of plasma membrane bounded cell projection assembly [GO:0120034]; positively regulates GO:0046847 Also known as: positive regulation of filopodia biosynthesis, positive regulation of filopodia formation, positive regulation of filopodium formation, up regulation of filopodium formation, up-regulation of filopodium formation, upregulation of filopodium formation, activation of filopodium formation, stimulation of filopodium formation